{
  "gene_name": "Dynactin-associated protein",
  "gene": "UniProtKB:Q8N1N2",
  "gene_symbol": "DYNAP",
  "term_id": "GO:0008284",
  "term_label": "positive regulation of cell population proliferation"
}